{
  "term_id": "GO:0008139",
  "term_label": "nuclear localization sequence binding",
  "gene_name": "Importin subunit alpha-6",
  "gene_symbol": "KPNA5",
  "gene": "UniProtKB:O15131"
}